{
  "term_id": "GO:0005634",
  "gene_symbol": "NEUROD6",
  "gene_name": "Neurogenic differentiation factor 6",
  "term_label": "nucleus",
  "gene": "UniProtKB:Q96NK8"
}